chitin synthase activity [GO:0004100] (MF) Also known as: UDP-N-acetyl-D-glucosamine:chitin 4-beta-N-acetylglucosaminyl-transferase activity, chitin synthetase activity, chitin-UDP N-acetylglucosaminyltransferase activity, chitin-UDP acetyl-glucosaminyl transferase activity, chitin-uridine diphosphate acetylglucosaminyltransferase activity, trans-N-acetylglucosaminosylase activity Definition: Catalysis of the reaction: UDP-N-acetyl-D-glucosamine + [->4)-N-acetyl-beta-D-glucosaminyl-(1-](n) = UDP + [->4)-N-acetyl-beta-D-glucosaminyl-(1-](n+1). Sources: EC:2.4.1.16 Relationships: is a type of GO:0008375